{
  "gene_symbol": "FUT4",
  "gene_name": "Alpha-(1,3)-fucosyltransferase 4",
  "gene": "UniProtKB:P22083",
  "term_id": "GO:0017083",
  "term_label": "4-galactosyl-N-acetylglucosaminide 3-alpha-L-fucosyltransferase activity"
}